{
  "gene_name": "Ras-related protein Rab-2A",
  "term_label": "Golgi apparatus",
  "gene_symbol": "RAB2A",
  "term_id": "GO:0005794",
  "gene": "UniProtKB:P61019"
}